{
  "term_label": "growth factor activity",
  "term_id": "GO:0008083",
  "gene_symbol": "AREG",
  "gene_name": "Amphiregulin",
  "gene": "UniProtKB:P15514"
}